{
  "gene_name": "Glycoprotein hormones alpha chain",
  "gene": "UniProtKB:P01215",
  "gene_symbol": "CGA",
  "term_id": "GO:0016914",
  "term_label": "follicle-stimulating hormone complex"
}